{
  "term_id": "UNKNOWN:0002",
  "gene": "UniProtKB:F8W0I5",
  "gene_name": "Nuclear pore complex-interacting protein family member B12",
  "term_label": "Unknown biological process",
  "gene_symbol": "NPIPB12"
}